{
  "gene": "UniProtKB:Q9UK45",
  "gene_symbol": "LSM7",
  "term_id": "GO:0071013",
  "gene_name": "U6 snRNA-associated Sm-like protein LSm7",
  "term_label": "catalytic step 2 spliceosome"
}